{
  "gene_name": "HEAT repeat-containing protein 3",
  "term_id": "UNKNOWN:0003",
  "gene_symbol": "HEATR3",
  "gene": "UniProtKB:Q7Z4Q2",
  "term_label": "Unknown cellular component"
}